{
  "gene_name": "PTPN13-like protein, Y-linked",
  "term_id": "UNKNOWN:0002",
  "gene_symbol": "PRYP4",
  "gene": "UniProtKB:O14603",
  "term_label": "Unknown biological process"
}